{
  "gene_name": "Retinoic acid receptor beta",
  "term_id": "GO:0090575",
  "gene": "UniProtKB:P10826",
  "term_label": "RNA polymerase II transcription regulator complex",
  "gene_symbol": "RARB"
}